{
  "gene": "UniProtKB:Q9NVP2",
  "gene_name": "Histone chaperone ASF1B",
  "gene_symbol": "ASF1B",
  "term_id": "GO:0000785",
  "term_label": "chromatin"
}